afferent axon development in lateral line nerve [GO:0048893] (biological process) Relationships: is a type of axon development [GO:0061564]; is part of lateral line nerve development [GO:0048892] Definition: The process whose specific outcome is the progression of an afferent axon in a lateral line nerve over time from its formation to the mature structure. This process includes axonogenesis and pathfinding of the afferent axons in any lateral line nerve. References: PMID:15832385 Subtypes: afferent axon development in anterior lateral line nerve [GO:0048910], afferent axon development in posterior lateral line nerve [GO:0048933]